{
  "term_id": "UNKNOWN:0001",
  "term_label": "Unknown molecular function",
  "gene_name": "Glycerol-3-phosphate acyltransferase 4",
  "gene": "UniProtKB:Q86UL3",
  "gene_symbol": "GPAT4"
}